{
  "gene_name": "Keratin, type I cytoskeletal 20",
  "gene": "UniProtKB:P35900",
  "gene_symbol": "KRT20",
  "term_label": "epithelial cell differentiation",
  "term_id": "GO:0030855"
}